{
  "term_label": "GTPase activity",
  "term_id": "GO:0003924",
  "gene_symbol": "ATL1",
  "gene_name": "Atlastin-1",
  "gene": "UniProtKB:Q8WXF7"
}